{
  "term_label": "structural constituent of cytoskeleton",
  "gene_name": "Desmin",
  "gene": "UniProtKB:P17661",
  "gene_symbol": "DES",
  "term_id": "GO:0005200"
}